DNA integrity checkpoint signaling [GO:0031570] (biological process) Also known as: DNA integrity checkpoint, signal transduction involved in DNA integrity checkpoint Sources: GOC:mtg_cell_cycle Relationships: is a type of cell cycle checkpoint signaling [GO:0000075] Subtypes: DNA replication checkpoint signaling [GO:0000076], DNA damage checkpoint signaling [GO:0000077], mitotic DNA integrity checkpoint signaling [GO:0044774], meiotic DNA integrity checkpoint signaling [GO:0044778] Definition: A signaling process that controls cell cycle progression in response to changes in DNA structure by monitoring the integrity of the DNA. The DNA integrity checkpoint begins with detection of DNA damage, defects in DNA structure or DNA replication, and progresses through signal transduction and ends with cell cycle effector processes.